{
  "gene_name": "Cancer_testis antigen family 45 member A2",
  "gene": "UniProtKB:Q5DJT8",
  "term_id": "UNKNOWN:0003",
  "term_label": "Unknown cellular component",
  "gene_symbol": "CT45A2"
}